{
  "term_id": "GO:0045766",
  "gene": "UniProtKB:P35590",
  "gene_name": "Tyrosine-protein kinase receptor Tie-1",
  "term_label": "positive regulation of angiogenesis",
  "gene_symbol": "TIE1"
}